pigment metabolic process [GO:0042440] (biological process) Also known as: pigment metabolism Subtypes: melanin metabolic process [GO:0006582], heme metabolic process [GO:0042168], pigment metabolic process involved in pigmentation [GO:0043474], GO:0046148, GO:0046149, anthocyanin-containing compound metabolic process [GO:0046283], flavone metabolic process [GO:0051552] Sources: GOC:jl, ISBN:0198506732 Relationships: is a type of metabolic process [GO:0008152] Definition: The chemical reactions and pathways involving pigment, any general or particular coloring matter in living organisms, e.g. melanin.